{
  "gene": "UniProtKB:Q96NX5",
  "gene_symbol": "CAMK1G",
  "gene_name": "Calcium_calmodulin-dependent protein kinase type 1G",
  "term_id": "GO:0005737",
  "term_label": "cytoplasm"
}